{
  "gene_symbol": "PSAPL1",
  "gene": "UniProtKB:Q6NUJ1",
  "term_id": "GO:0060742",
  "term_label": "epithelial cell differentiation involved in prostate gland development",
  "gene_name": "Proactivator polypeptide-like 1"
}